negative regulation of fast-twitch skeletal muscle fiber contraction [GO:0031447] (biological process) Relationships: is_a regulation of fast-twitch skeletal muscle fiber contraction [GO:0031446]; is a type of negative regulation of striated muscle contraction [GO:0045988]; negatively regulates fast-twitch skeletal muscle fiber contraction [GO:0031443] Definition: Any process that stops, prevents, or reduces the frequency, rate or extent of fast-twitch skeletal muscle contraction. Sources: GOC:dph, GOC:ef, GOC:mah, GOC:mtg_muscle, GOC:tb Also known as: down regulation of fast-twitch skeletal muscle contraction, down-regulation of fast-twitch skeletal muscle contraction, downregulation of fast-twitch skeletal muscle contraction, negative regulation of fast-twitch skeletal muscle contraction, inhibition of fast-twitch skeletal muscle contraction